{
  "gene_name": "Zinc finger E-box-binding homeobox 2",
  "gene": "UniProtKB:O60315",
  "gene_symbol": "ZEB2",
  "term_id": "GO:0007417",
  "term_label": "central nervous system development"
}